{
  "term_label": "protein serine/threonine kinase activator activity",
  "gene": "UniProtKB:Q8TAI7",
  "gene_symbol": "RHEBL1",
  "term_id": "GO:0043539",
  "gene_name": "GTPase RhebL1"
}